negative regulation of amino acid transport [GO:0051956] (BP) Definition: Any process that stops, prevents, or reduces the frequency, rate or extent of the directed movement of amino acids into, out of or within a cell, or between cells, by means of some agent such as a transporter or pore. Sources: GOC:ai Also known as: down regulation of amino acid transport, down-regulation of amino acid transport, downregulation of amino acid transport, negative regulation of amino acid transmembrane transport, inhibition of amino acid transport Relationships: is a type of negative regulation of amine transport [GO:0051953]; is a type of regulation of amino acid transport [GO:0051955]; negatively regulates amino acid transport [GO:0006865] Subtypes: negative regulation of L-glutamate import across plasma membrane [GO:0002037], negative regulation of glutamate secretion [GO:0014050], negative regulation of gamma-aminobutyric acid secretion [GO:0014053], negative regulation of amino acid uptake involved in synaptic transmission [GO:0051942], GO:0140216, negative regulation of glycine import across plasma membrane [GO:1900924], negative regulation of L-threonine import across plasma membrane [GO:1900927], GO:1900930, negative regulation of proline import across plasma membrane [GO:1902835], negative regulation of aspartate secretion [GO:1904449], negative regulation of glycine secretion, neurotransmission [GO:1904625], negative regulation of L-lysine import across plasma membrane [GO:1905009], negative regulation of L-leucine import across plasma membrane [GO:1905533], GO:1905542, negative regulation of L-methionine import across plasma membrane [GO:1905625], negative regulation of glutamine transport [GO:2000486]